interleukin-3 receptor binding [GO:0005135] (molecular function) Definition: Binding to an interleukin-3 receptor. Sources: GOC:ai Also known as: IL-3, interleukin-3 receptor ligand Relationships: is a type of GO:0005126; is a type of GO:0070851